{
  "gene": "UniProtKB:Q13253",
  "term_id": "GO:0030514",
  "gene_symbol": "NOG",
  "term_label": "negative regulation of BMP signaling pathway",
  "gene_name": "Noggin"
}